craniofacial suture morphogenesis [GO:0097094] (biological process) Subtypes: cranial suture morphogenesis [GO:0060363], frontonasal suture morphogenesis [GO:0097095], facial suture morphogenesis [GO:0097096] Relationships: is_a anatomical structure morphogenesis [GO:0009653]; BFO_0000050 bone morphogenesis [GO:0060349]; is part of cranial skeletal system development [GO:1904888] Definition: The process in which any suture between cranial and/or facial bones is generated and organized. Sources: GOC:pr, GOC:sl, Wikipedia:Cranial_sutures, Wikipedia:Head_and_neck_anatomy#Musculoskeletal_system